{
  "term_label": "microtubule organizing center",
  "gene_symbol": "CCNB2",
  "gene": "UniProtKB:O95067",
  "term_id": "GO:0005815",
  "gene_name": "G2_mitotic-specific cyclin-B2"
}